{
  "gene_name": "Tau-tubulin kinase 1",
  "term_id": "GO:0005737",
  "gene_symbol": "TTBK1",
  "gene": "UniProtKB:Q5TCY1",
  "term_label": "cytoplasm"
}